positive regulation of neuronal signal transduction [GO:1902849] (biological process) Definition: Any process that activates or increases the frequency, rate or extent of neuronal signal transduction. Also known as: up regulation of neuronal signal transduction, up-regulation of neuronal signal transduction, upregulation of neuronal signal transduction, activation of neuronal signal transduction Relationships: is a type of positive regulation of signal transduction [GO:0009967]; is a type of regulation of neuronal signal transduction [GO:1902847]; positively regulates neuronal signal transduction [GO:0023041] Sources: GOC:TermGenie, GOC:sjp, GO_REF:0000058